{
  "term_id": "UNKNOWN:0001",
  "gene_name": "Biorientation of chromosomes in cell division protein 1-like 2",
  "term_label": "Unknown molecular function",
  "gene": "UniProtKB:Q8IYS8",
  "gene_symbol": "BOD1L2"
}